cytochrome-c3 hydrogenase activity [GO:0047806] (MF) Relationships: is a type of oxidoreductase activity, acting on hydrogen as donor, cytochrome as acceptor [GO:0016697] Definition: Catalysis of the reaction: 2 H2 + ferricytochrome c3 = 4 H+ + ferrocytochrome c3. Also known as: cytochrome hydrogenase activity, H(2):ferricytochrome c3 oxidoreductase activity, H2:ferricytochrome c3 oxidoreductase activity, cytochrome c3 reductase activity, hydrogen:ferricytochrome-c3 oxidoreductase activity Sources: EC:1.12.2.1, MetaCyc:CYTOCHROME-C3-HYDROGENASE-RXN